atrial cardiac muscle cell-AV node cell adhesion involved in cell communication [GO:0086071] (biological process) Also known as: atrial cardiomyocyte-AV node cell adhesion involved in cell communication, atrial cardiomyocyte-atrioventricular node cell adhesion involved in cell communication Definition: The attachment of an atrial cardiomyocyte to an AV node cell via adhesion molecules that results in the cells being juxtaposed so that they can communicate. Sources: GOC:BHF, GOC:mtg_cardiac_conduct_nov11 Relationships: is a type of heterotypic cell-cell adhesion [GO:0034113]; is a type of cardiac muscle cell-cardiac muscle cell adhesion [GO:0086042]; BFO_0000050 atrial cardiac muscle cell to AV node cell communication [GO:0086066]